{
  "gene_symbol": "VTI1A",
  "gene_name": "Vesicle transport through interaction with t-SNAREs homolog 1A",
  "gene": "UniProtKB:Q96AJ9",
  "term_label": "late endosome membrane",
  "term_id": "GO:0031902"
}